{
  "term_id": "GO:0005829",
  "gene": "UniProtKB:P10644",
  "gene_name": "cAMP-dependent protein kinase type I-alpha regulatory subunit",
  "gene_symbol": "PRKAR1A",
  "term_label": "cytosol"
}